leukocyte mediated immunity [GO:0002443] (biological process) Definition: Any process involved in the carrying out of an immune response by a leukocyte. Regulation: regulated by GO:0002703; negatively regulated by GO:0002704; RO_0002213 by positive regulation of leukocyte mediated immunity [GO:0002705] Sources: GOC:add, GO_REF:0000022, ISBN:0781735149 Relationships: is a type of immune effector process [GO:0002252] Also known as: immune cell effector process, immune cell mediated immunity, leucocyte immune effector process, leucocyte mediated immunity, leukocyte immune effector process, cell-mediated immune response, cellular immune response Subtypes: GO:0001909, dendritic cell cytokine production [GO:0002371], myeloid leukocyte mediated immunity [GO:0002444], lymphocyte mediated immunity [GO:0002449]